{
  "gene_name": "Left-right determination factor 2",
  "gene_symbol": "LEFTY2",
  "term_label": "cytokine activity",
  "gene": "UniProtKB:O00292",
  "term_id": "GO:0005125"
}